steroid hydroxylase activity [GO:0008395] (MF) Sources: ISBN:0721662544 Relationships: is a type of GO:0004497 Definition: Catalysis of the formation of a hydroxyl group on a steroid by incorporation of oxygen from O2. Also known as: steroid monooxygenase activity, cytochrome P450 CYP2G1, olfactory-specific steroid hydroxylase activity Subtypes: GO:0001567, GO:0004501, GO:0004507, GO:0004508, GO:0004509, cholesterol monooxygenase (side-chain-cleaving) activity [GO:0008386], GO:0008387, steroid 15-alpha-hydroxylase activity [GO:0008388], testosterone 16-alpha-hydroxylase activity [GO:0008390], sterol 12-alpha-hydroxylase activity [GO:0008397], GO:0030343, GO:0031073, ecdysteroid 25-hydroxylase activity [GO:0035302], GO:0042767, ecdysteroid 2-hydroxylase activity [GO:0042768], GO:0047882, progesterone monooxygenase activity [GO:0050214], steroid 9-alpha-monooxygenase activity [GO:0050292], GO:0050649, GO:0062179, testosterone 16-beta-hydroxylase activity [GO:0062184], vitamin D 24-hydroxylase activity [GO:0070576], estrogen 16-alpha-hydroxylase activity [GO:0101020], GO:0101021, GO:0160191